mitochondrial protein quality control [GO:0141164] (biological process) Relationships: is a type of protein quality control for misfolded or incompletely synthesized proteins [GO:0006515] References: PMID:38280230 Definition: The chemical reactions and pathways resulting in the breakdown of misfolded proteins in the mitochondrion, which are targeted for degradation.